sperm cytoplasmic droplet [GO:0097598] (cellular component) Relationships: is a type of cytoplasmic vesicle [GO:0031410] Definition: A small amount of cytoplasm surrounded by a cell membrane that is generally retained in spermatozoa after spermiogenesis, when the majority of the cytoplasm is phagocytosed by Sertoli cells to produce what are called residual bodies. Initially, the droplet is located at the neck just behind the head of an elongated spermatid. During epididymal transit, the cytoplasmic droplet migrates caudally to the annulus at the end of the midpiece; the exact position and time varies by species. The cytoplasmic droplet consists of lipids, lipoproteins, RNAs, a variety of hydrolytic enzymes, receptors, ion channels, and Golgi-derived vesicles. The droplet may be involved in regulatory volume loss (RVD) at ejaculation, and in most species, though not in humans, the cytoplasmic droplet is lost at ejaculation. Note that the cytoplasmic droplet is distinct from 'excessive residual cytoplasm' that sometimes remains in epididymal spermatozoa, particularly when spermiogenesis has been disrupted. References: PMID:12672117, PMID:21076437, PMID:23159014 Sources: GOC:krc, GOC:vesicles Also known as: sperm residual cytoplasm